{
  "term_id": "GO:0006338",
  "gene_symbol": "KDM5B",
  "gene_name": "Lysine-specific demethylase 5B",
  "term_label": "chromatin remodeling",
  "gene": "UniProtKB:Q9UGL1"
}